beta-2 adrenergic receptor binding [GO:0031698] (molecular function) Relationships: is a type of adrenergic receptor binding [GO:0031690] Definition: Binding to a beta-2 adrenergic receptor. Also known as: beta-2 adrenergic receptor ligand Sources: GOC:mah, GOC:nln